{
  "term_id": "GO:0030036",
  "term_label": "actin cytoskeleton organization",
  "gene": "UniProtKB:O60890",
  "gene_symbol": "OPHN1",
  "gene_name": "Oligophrenin-1"
}